{
  "gene_name": "N-acylneuraminate-9-phosphatase",
  "gene_symbol": "NANP",
  "term_label": "N-acetylneuraminate biosynthetic process",
  "gene": "UniProtKB:Q8TBE9",
  "term_id": "GO:0046380"
}